{
  "gene_symbol": "POMC",
  "term_id": "GO:0005615",
  "gene_name": "Pro-opiomelanocortin",
  "gene": "UniProtKB:P01189",
  "term_label": "extracellular space"
}